peptidoglycan biosynthetic process [GO:0009252] (biological process) Definition: The chemical reactions and pathways resulting in the formation of peptidoglycans, any of a class of glycoconjugates found in bacterial cell walls and consisting of long glycan strands of alternating residues of beta-(1,4) linked N-acetylglucosamine and N-acetylmuramic acid, cross-linked by short peptides. Also known as: murein biosynthesis, murein biosynthetic process, peptidoglycan anabolism, peptidoglycan biosynthesis, peptidoglycan formation, peptidoglycan synthesis Relationships: is_a peptidoglycan metabolic process [GO:0000270]; is a type of glycosaminoglycan biosynthetic process [GO:0006024]; is a type of GO:0044038; is part of GO:0009273 Subtypes: peptidoglycan-protein cross-linking [GO:0018104] References: PMID:18266853